{
  "term_label": "olfactory receptor activity",
  "term_id": "GO:0004984",
  "gene_symbol": "OR2K2",
  "gene_name": "Olfactory receptor 2K2",
  "gene": "UniProtKB:Q8NGT1"
}